peptide antigen binding [GO:0042605] (molecular function) Sources: GOC:add, GOC:jl, GOC:rv Also known as: endogenous peptide antigen binding, exogenous peptide antigen binding Note: Note that this term can be used to describe the binding of a peptide to an MHC molecule. Relationships: is a type of GO:0003823; is_a peptide binding [GO:0042277] Definition: Binding to an antigen peptide.